{
  "gene": "UniProtKB:A0A075B6H5",
  "gene_symbol": "TRBV20OR9-2",
  "term_id": "UNKNOWN:0001",
  "gene_name": "T cell receptor beta variable 20_OR9-2 (non-functional) (Fragment)",
  "term_label": "Unknown molecular function"
}